{
  "gene_name": "ATP synthase subunit alpha, mitochondrial",
  "gene": "UniProtKB:P25705",
  "term_label": "proton-transporting ATP synthase activity, rotational mechanism",
  "gene_symbol": "ATP5F1A",
  "term_id": "GO:0046933"
}